phosphatidylinositol-mediated signaling [GO:0048015] (biological process) Sources: GOC:bf, GOC:ceb, ISBN:0198506732 Definition: The series of molecular signals in which a cell uses a phosphatidylinositol-mediated signaling to convert a signal into a response. Phosphatidylinositols include phosphatidylinositol (PtdIns) and its phosphorylated derivatives. Also known as: inositol phospholipid-mediated signaling, phosphatidylinositol-mediated signal transduction, phosphatidylinositol-mediated signalling, phosphoinositide-mediated signaling, phosphoinositide-mediated signalling Relationships: is a type of intracellular signal transduction [GO:0035556]